beta-D-glucose oxidase activity [GO:0046562] (molecular function) Sources: RHEA:11428 Also known as: glucose oxidase activity, D-glucose oxidase activity, D-glucose-1-oxidase activity, GOD activity, beta-D-glucose:oxygen 1-oxido-reductase activity, beta-D-glucose:oxygen 1-oxidoreductase activity, beta-D-glucose:quinone oxidoreductase activity, corylophyline, deoxin-1, glucose aerodehydrogenase activity, glucose oxyhydrase activity, microcid, penatin Definition: Catalysis of the reaction: beta-D-glucose + O2 = D-glucono-1,5-lactone + H2O2. Relationships: is a type of hexose oxidase activity [GO:0047979]